{
  "gene_symbol": "BAK1",
  "gene": "UniProtKB:Q16611",
  "gene_name": "Bcl-2 homologous antagonist_killer",
  "term_id": "GO:0001836",
  "term_label": "release of cytochrome c from mitochondria"
}